{
  "term_label": "Unknown biological process",
  "gene_name": "Arylsulfatase K",
  "gene_symbol": "ARSK",
  "gene": "UniProtKB:Q6UWY0",
  "term_id": "UNKNOWN:0002"
}